{
  "gene_name": "Ras-GEF domain-containing family member 1B",
  "term_id": "GO:0005886",
  "gene_symbol": "RASGEF1B",
  "term_label": "plasma membrane",
  "gene": "UniProtKB:Q0VAM2"
}